{
  "gene": "UniProtKB:Q5SZB4",
  "term_label": "Unknown cellular component",
  "gene_symbol": "C9orf50",
  "gene_name": "Uncharacterized protein C9orf50",
  "term_id": "UNKNOWN:0003"
}